{
  "gene_name": "Protein phosphatase Slingshot homolog 3",
  "term_label": "actin cytoskeleton organization",
  "gene": "UniProtKB:Q8TE77",
  "gene_symbol": "SSH3",
  "term_id": "GO:0030036"
}